{
  "gene_symbol": "OR3A2",
  "gene_name": "Olfactory receptor 3A2",
  "term_id": "GO:0004984",
  "gene": "UniProtKB:P47893",
  "term_label": "olfactory receptor activity"
}